{
  "term_label": "nucleus",
  "gene_symbol": "CDY2A",
  "gene": "UniProtKB:Q9Y6F7",
  "gene_name": "Testis-specific chromodomain protein Y 2",
  "term_id": "GO:0005634"
}